oxidoreductase activity, acting on single donors with incorporation of molecular oxygen, incorporation of one atom of oxygen (internal monooxygenases or internal mixed function oxidases) [GO:0016703] (molecular function) Sources: EC:1.13.12.-, GOC:mah Relationships: is a type of GO:0004497; is a type of oxidoreductase activity, acting on single donors with incorporation of molecular oxygen [GO:0016701] Definition: Catalysis of an oxidation-reduction (redox) reaction in which hydrogen or electrons are transferred from one donor, and one oxygen atom is incorporated into a donor. Subtypes: chlorophyllide a oxygenase activity [GO:0010277], nitronate monooxygenase activity [GO:0018580], Oplophorus-luciferin 2-monooxygenase activity [GO:0033756], GO:0036434, GO:0047077, L-lysine 6-monooxygenase (NADPH) activity [GO:0047091], arginine 2-monooxygenase activity [GO:0047678], Cypridina-luciferin 2-monooxygenase activity [GO:0047712], lactate 2-monooxygenase activity [GO:0050040], GO:0050067, phenylalanine 2-monooxygenase activity [GO:0050172], GO:0050248, GO:0050361, Watasenia-luciferin 2-monooxygenase activity [GO:0050397], apo-beta-carotenoid-14',13'-dioxygenase activity [GO:0050588], 2-oxoglutarate oxygenase/decarboxylase (ethylene-forming) activity [GO:0102276], 1,3,6,8-tetrahydroxynaphthalene monooxygenase (quinone-forming) activity [GO:0102634], GO:0102818